{
  "gene_symbol": "GOLGA6D",
  "term_label": "Golgi organization",
  "gene": "UniProtKB:P0CG33",
  "gene_name": "Golgin subfamily A member 6D",
  "term_id": "GO:0007030"
}